{
  "gene_symbol": "FLT3",
  "term_label": "positive regulation of cell population proliferation",
  "gene": "UniProtKB:P36888",
  "gene_name": "Receptor-type tyrosine-protein kinase FLT3",
  "term_id": "GO:0008284"
}